{
  "gene_name": "Gamma-aminobutyric acid receptor subunit gamma-2",
  "gene_symbol": "GABRG2",
  "term_id": "GO:1902476",
  "term_label": "chloride transmembrane transport",
  "gene": "UniProtKB:P18507"
}